tryptophan-tRNA ligase activity [GO:0004830] (molecular function) Definition: Catalysis of the reaction: ATP + L-tryptophan + tRNA(Trp) = AMP + diphosphate + L-tryptophanyl-tRNA(Trp). Relationships: is a type of aminoacyl-tRNA ligase activity [GO:0004812] Sources: EC:6.1.1.2 Also known as: tryptophanyl-tRNA synthetase activity, L-tryptophan-tRNA(Trp) ligase (AMP-forming) activity, L-tryptophan-tRNATrp ligase (AMP-forming), L-tryptophan:tRNATrp ligase (AMP-forming), TrpRS activity, tryptophan translase activity, tryptophanyl ribonucleic synthetase activity, tryptophanyl-tRNA synthase activity, tryptophanyl-transfer RNA synthetase activity, tryptophanyl-transfer ribonucleate synthetase activity, tryptophanyl-transfer ribonucleic acid synthetase activity, tryptophanyl-transfer ribonucleic synthetase activity